{
  "term_id": "GO:0016020",
  "term_label": "membrane",
  "gene": "UniProtKB:Q96MH6",
  "gene_name": "Monoacylglycerol_Diacylglycerol O-acyltransferase",
  "gene_symbol": "TMEM68"
}